{
  "term_id": "GO:0005615",
  "gene_symbol": "ANPEP",
  "gene": "UniProtKB:P15144",
  "gene_name": "Aminopeptidase N",
  "term_label": "extracellular space"
}